negative regulation of mitotic metaphase/anaphase transition [GO:0045841] (biological process) Also known as: down regulation of mitotic metaphase/anaphase transition, down-regulation of mitotic metaphase/anaphase transition, downregulation of mitotic metaphase/anaphase transition, inhibition of mitotic metaphase/anaphase transition Definition: Any process that stops, prevents, or reduces the frequency, rate or extent of the cell cycle process in which a cell progresses from metaphase to anaphase during mitosis, triggered by the activation of the anaphase promoting complex by Cdc20/Sleepy homolog which results in the degradation of Securin. Sources: GOC:go_curators Subtypes: mitotic spindle assembly checkpoint signaling [GO:0007094] Relationships: is a type of regulation of mitotic metaphase/anaphase transition [GO:0030071]; is a type of negative regulation of mitotic nuclear division [GO:0045839]; is a type of negative regulation of mitotic cell cycle phase transition [GO:1901991]; is a type of GO:1902100; is a type of negative regulation of mitotic sister chromatid separation [GO:2000816]; negatively regulates metaphase/anaphase transition of mitotic cell cycle [GO:0007091]